{
  "gene_name": "Forkhead box protein N4",
  "term_label": "DNA-binding transcription factor activity",
  "gene_symbol": "FOXN4",
  "term_id": "GO:0003700",
  "gene": "UniProtKB:Q96NZ1"
}